anastral spindle assembly [GO:0055048] (biological process) Definition: The aggregation, arrangement and bonding together of a set of components to form the spindle, the array of microtubules and associated molecules that serves to move duplicated chromosomes apart, in the absence of centrosomes. Formation is initiated by the nucleation of microtubules (MTs) in the vicinity of condensed chromatin. MTs then attach to and congress around the chromatin due to activity of microtubule motors. A bipolar spindle is formed by focusing of the terminal ends of the MT array into spindle poles by molecular motors and cross-linking proteins. References: PMID:15034926 Sources: GOC:expert_rg, GOC:mtg_sensu, GOC:tb Relationships: is a type of spindle assembly [GO:0051225] Subtypes: anastral spindle assembly involved in male meiosis [GO:0009971]